{
  "gene": "UniProtKB:O60504",
  "gene_name": "Vinexin",
  "gene_symbol": "SORBS3",
  "term_label": "nucleus",
  "term_id": "GO:0005634"
}